centromeric DNA binding [GO:0019237] (molecular function) Also known as: centromere binding Sources: GOC:jl, SO:0000577 Definition: Binding to a centromere, a region of chromosome where the spindle fibers attach during mitosis and meiosis. Relationships: is a type of sequence-specific double-stranded DNA binding [GO:1990837]